{
  "term_label": "Unknown molecular function",
  "term_id": "UNKNOWN:0001",
  "gene_symbol": "SCAND3",
  "gene": "UniProtKB:Q6R2W3",
  "gene_name": "SCAN domain-containing protein 3"
}